{
  "term_label": "plasma membrane",
  "gene_name": "Complement component 1 Q subcomponent-binding protein, mitochondrial",
  "gene_symbol": "C1QBP",
  "gene": "UniProtKB:Q07021",
  "term_id": "GO:0005886"
}